{
  "term_label": "transcription corepressor activity",
  "gene": "UniProtKB:Q8N108",
  "term_id": "GO:0003714",
  "gene_name": "Mesoderm induction early response protein 1",
  "gene_symbol": "MIER1"
}